tRNA nucleotidyltransferase activity [GO:0009022] (molecular function) Note: Note that, although EC names the enzme tRNA nucleotidyltransferase, the enzyme to which this term refers is also known as 'ribonuclease PH', and degrades tRNA in the 3'-5' direction in vivo. It should not be confused with CCA tRNA nucleotidyltransferase. References: PMID:2455297 Sources: RHEA:10628 Definition: Catalysis of the reaction: tRNA(n+1) + phosphate = tRNA(n) + a nucleoside diphosphate. Also known as: RNase PH activity, phosphate-dependent exonuclease activity, ribonuclease PH activity Relationships: is a type of GO:0016779; is a type of catalytic activity, acting on a tRNA [GO:0140101]